{
  "term_id": "GO:0097060",
  "gene": "UniProtKB:Q5VT97",
  "gene_name": "Rho GTPase-activating protein SYDE2",
  "gene_symbol": "SYDE2",
  "term_label": "synaptic membrane"
}